negative regulation of type 2 immune response [GO:0002829] (biological process) Sources: GOC:add Relationships: is a type of regulation of type 2 immune response [GO:0002828]; is a type of negative regulation of immune response [GO:0050777]; negatively regulates type 2 immune response [GO:0042092] Subtypes: negative regulation of T-helper 2 cell differentiation [GO:0045629], negative regulation of T-helper 2 cell cytokine production [GO:2000552] Definition: Any process that stops, prevents, or reduces the frequency, rate, or extent of a type 2 immune response. Also known as: down regulation of type 2 immune response, down-regulation of type 2 immune response, downregulation of type 2 immune response, inhibition of type 2 immune response, negative regulation of T-helper 2 type immune response, negative regulation of Th2 immune response